{
  "gene_name": "Protein regulator of cytokinesis 1",
  "gene": "UniProtKB:O43663",
  "term_id": "GO:0005819",
  "term_label": "spindle",
  "gene_symbol": "PRC1"
}